{
  "term_label": "RNA polymerase II cis-regulatory region sequence-specific DNA binding",
  "gene_symbol": "NKX2-6",
  "gene_name": "Homeobox protein Nkx-2.6",
  "gene": "UniProtKB:A6NCS4",
  "term_id": "GO:0000978"
}